{
  "gene_name": "T-box transcription factor TBX15",
  "term_id": "GO:0000785",
  "term_label": "chromatin",
  "gene_symbol": "TBX15",
  "gene": "UniProtKB:Q96SF7"
}